{
  "gene": "UniProtKB:Q9NSD4",
  "gene_name": "Zinc finger protein 275",
  "term_label": "regulation of transcription by RNA polymerase II",
  "term_id": "GO:0006357",
  "gene_symbol": "ZNF275"
}